{
  "term_label": "Unknown molecular function",
  "term_id": "UNKNOWN:0001",
  "gene_name": "Bcl-2-like protein 11",
  "gene_symbol": "BCL2L11",
  "gene": "UniProtKB:O43521"
}